{
  "term_id": "UNKNOWN:0002",
  "gene_name": "Uncharacterized protein C10orf120",
  "gene_symbol": "C10orf120",
  "term_label": "Unknown biological process",
  "gene": "UniProtKB:Q5SQS8"
}